{
  "gene_symbol": "BRD9",
  "term_id": "GO:0140566",
  "gene": "UniProtKB:Q9H8M2",
  "gene_name": "Bromodomain-containing protein 9",
  "term_label": "histone reader activity"
}